{
  "gene": "UniProtKB:Q13283",
  "term_label": "cytoplasmic stress granule",
  "gene_name": "Ras GTPase-activating protein-binding protein 1",
  "term_id": "GO:0010494",
  "gene_symbol": "G3BP1"
}